negative regulation of L-dopa biosynthetic process [GO:1903196] (biological process) Sources: GOC:PARL, GOC:TermGenie, GOC:bf, GO_REF:0000058 Also known as: down regulation of L-dopa anabolism, down regulation of L-dopa biosynthesis, down regulation of L-dopa biosynthetic process, down regulation of L-dopa formation, down regulation of L-dopa synthesis, down-regulation of L-dopa anabolism, down-regulation of L-dopa biosynthesis, down-regulation of L-dopa biosynthetic process, down-regulation of L-dopa formation, down-regulation of L-dopa synthesis, downregulation of L-dopa anabolism, downregulation of L-dopa biosynthesis, downregulation of L-dopa biosynthetic process, downregulation of L-dopa formation, downregulation of L-dopa synthesis, negative regulation of L-dopa anabolism, negative regulation of L-dopa biosynthesis, negative regulation of L-dopa formation, negative regulation of L-dopa synthesis, inhibition of L-dopa anabolism, inhibition of L-dopa biosynthesis, inhibition of L-dopa biosynthetic process, inhibition of L-dopa formation, inhibition of L-dopa synthesis Relationships: is a type of negative regulation of small molecule metabolic process [GO:0062014]; is a type of regulation of L-dopa biosynthetic process [GO:1903195]; is_a negative regulation of amino acid biosynthetic process [GO:2000283]; negatively regulates GO:1903185 Definition: Any process that stops, prevents or reduces the frequency, rate or extent of L-dopa biosynthetic process.